{
  "gene_symbol": "MT1E",
  "gene_name": "Metallothionein-1E",
  "gene": "UniProtKB:P04732",
  "term_id": "GO:0071276",
  "term_label": "cellular response to cadmium ion"
}